aristolochene synthase activity [GO:0045483] (molecular function) Sources: EC:4.2.3.9 Also known as: sesquiterpene cyclase activity, 2-trans,6-trans-farnesyl-diphosphate diphosphate-lyase (cyclizing, aristolochene-forming), trans,trans-farnesyl diphosphate aristolochene-lyase activity, trans,trans-farnesyl-diphosphate diphosphate-lyase (cyclizing, aristolochene-forming) Definition: Catalysis of the reaction: trans,trans-farnesyl diphosphate = aristolochene + diphosphate. Relationships: is a type of sesquiterpene synthase activity [GO:0010334]